{
  "term_id": "GO:0003712",
  "gene_symbol": "MED26",
  "term_label": "transcription coregulator activity",
  "gene": "UniProtKB:O95402",
  "gene_name": "Mediator of RNA polymerase II transcription subunit 26"
}